{
  "term_label": "NF-kappaB binding",
  "term_id": "GO:0051059",
  "gene_symbol": "FAF1",
  "gene_name": "FAS-associated factor 1",
  "gene": "UniProtKB:Q9UNN5"
}